{
  "gene": "UniProtKB:Q99075",
  "term_id": "GO:0005615",
  "term_label": "extracellular space",
  "gene_name": "Proheparin-binding EGF-like growth factor",
  "gene_symbol": "HBEGF"
}